{
  "gene": "UniProtKB:Q9Y487",
  "term_label": "ATPase binding",
  "term_id": "GO:0051117",
  "gene_name": "V-type proton ATPase 116 kDa subunit a 2",
  "gene_symbol": "ATP6V0A2"
}